{
  "gene": "UniProtKB:Q8N531",
  "gene_name": "F-box_LRR-repeat protein 6",
  "gene_symbol": "FBXL6",
  "term_label": "Unknown molecular function",
  "term_id": "UNKNOWN:0001"
}